{
  "term_id": "GO:1902626",
  "gene": "UniProtKB:P56537",
  "gene_symbol": "EIF6",
  "gene_name": "Eukaryotic translation initiation factor 6",
  "term_label": "assembly of large subunit precursor of preribosome"
}